{
  "gene_name": "ATP-dependent RNA helicase SUPV3L1, mitochondrial",
  "term_id": "GO:0045025",
  "term_label": "mitochondrial degradosome",
  "gene_symbol": "SUPV3L1",
  "gene": "UniProtKB:Q8IYB8"
}